{
  "gene": "UniProtKB:P35225",
  "gene_name": "Interleukin-13",
  "term_label": "extracellular space",
  "gene_symbol": "IL13",
  "term_id": "GO:0005615"
}